{
  "term_id": "UNKNOWN:0003",
  "gene": "UniProtKB:Q8NC24",
  "term_label": "Unknown cellular component",
  "gene_symbol": "RELL2",
  "gene_name": "RELT-like protein 2"
}